beta-amyrin synthase activity [GO:0042300] (molecular function) References: PMID:9746369 Sources: RHEA:31007 Relationships: is a type of oxidosqualene cyclase activity [GO:0031559] Definition: Catalysis of the reaction: (S)-2,3-epoxysqualene = beta-amyrin. Also known as: 2,3-oxidosqualene beta-amyrin cyclase, oxidosqualene:beta-amyrin cyclase activity